{
  "term_id": "GO:0044389",
  "gene_name": "Protein mono-ADP-ribosyltransferase PARP9",
  "term_label": "ubiquitin-like protein ligase binding",
  "gene_symbol": "PARP9",
  "gene": "UniProtKB:Q8IXQ6"
}